{
  "term_id": "UNKNOWN:0003",
  "term_label": "Unknown cellular component",
  "gene_name": "DNA-binding protein SATB1",
  "gene_symbol": "SATB1",
  "gene": "UniProtKB:Q01826"
}